2'-deoxyribonucleotide biosynthetic process [GO:0009265] (BP) Relationships: is a type of deoxyribonucleotide biosynthetic process [GO:0009263]; is a type of 2'-deoxyribonucleotide metabolic process [GO:0009394]; is a type of deoxyribose phosphate biosynthetic process [GO:0046385] Definition: The chemical reactions and pathways resulting in the formation of a 2'-deoxyribonucleotide, a compound consisting of 2'-deoxyribonucleoside (a base linked to a 2'-deoxyribose sugar) esterified with a phosphate group at either the 3' or 5'-hydroxyl group of the sugar. Also known as: 2'-deoxyribonucleotide anabolism, 2'-deoxyribonucleotide biosynthesis, 2'-deoxyribonucleotide formation, 2'-deoxyribonucleotide synthesis Sources: GOC:mah Subtypes: GO:0009153, pyrimidine deoxyribonucleotide biosynthetic process [GO:0009221]